{
  "gene_symbol": "ATP6V0E2",
  "gene": "UniProtKB:Q8NHE4",
  "term_id": "GO:1902600",
  "term_label": "proton transmembrane transport",
  "gene_name": "V-type proton ATPase subunit e 2"
}